{
  "term_label": "mediator complex",
  "gene_symbol": "UXT",
  "gene": "UniProtKB:Q9UBK9",
  "term_id": "GO:0016592",
  "gene_name": "Protein UXT"
}